{
  "term_label": "positive regulation of cytosolic calcium ion concentration",
  "gene_name": "Protachykinin-1",
  "gene_symbol": "TAC1",
  "term_id": "GO:0007204",
  "gene": "UniProtKB:P20366"
}